{
  "term_label": "centrosome cycle",
  "gene_name": "Partitioning defective 6 homolog beta",
  "term_id": "GO:0007098",
  "gene_symbol": "PARD6B",
  "gene": "UniProtKB:Q9BYG5"
}